calcium-dependent phospholipase A2 activity [GO:0047498] (molecular function) Definition: Catalysis of the reaction: phosphatidylcholine + H2O = 1-acylglycerophosphocholine + a carboxylate. This reaction requires Ca2+. Also known as: calcium-dependent cytosolic phospholipase A2 activity, calcium-dependent secreted phospholipase A2 activity References: PMID:34831185 Relationships: is a type of GO:0004623